UDP-glucose transmembrane transport [GO:0015786] (biological process) Sources: GOC:ai Definition: The process in which UDP-glucose is transported across a membrane. Subtypes: UDP-glucose transmembrane transport into endoplasmic reticulum [GO:0120112] Relationships: is a type of organic anion transport [GO:0015711]; is a type of pyrimidine nucleotide-sugar transmembrane transport [GO:0090481]